{
  "term_label": "glycine transmembrane transporter activity",
  "term_id": "GO:0015187",
  "gene": "UniProtKB:Q96DW6",
  "gene_name": "Mitochondrial glycine transporter",
  "gene_symbol": "SLC25A38"
}